{
  "gene_symbol": "ZNF93",
  "gene_name": "Zinc finger protein 93",
  "term_label": "RNA polymerase II cis-regulatory region sequence-specific DNA binding",
  "term_id": "GO:0000978",
  "gene": "UniProtKB:P35789"
}